{
  "term_id": "UNKNOWN:0001",
  "gene_symbol": "SNHG28",
  "term_label": "Unknown molecular function",
  "gene_name": "Putative uncharacterized protein SNHG28",
  "gene": "UniProtKB:P0DPA3"
}